{
  "gene_name": "WD repeat-containing protein 43",
  "term_label": "nucleolus",
  "gene": "UniProtKB:Q15061",
  "gene_symbol": "WDR43",
  "term_id": "GO:0005730"
}